inward rectifier potassium channel complex [GO:1902937] (cellular component) Note: An example of this is Kcnj2 in mouse (P35561) in PMID:16834334 (inferred from direct assay). Subtypes: GO:1990374, GO:1990566 Relationships: is_a voltage-gated potassium channel complex [GO:0008076] References: PMID:16834334 Sources: GOC:TermGenie, GOC:bhm, GO_REF:0000088 Definition: A protein complex which is capable of inward rectifier potassium channel activity.